negative regulation of mitochondrial calcium ion concentration [GO:0051562] (biological process) Also known as: mitochondrial calcium ion concentration reduction, reduction of calcium ion concentration in mitochondria, reduction of calcium ion concentration in mitochondrion, reduction of mitochondrial calcium ion concentration Relationships: is a type of mitochondrial calcium ion homeostasis [GO:0051560] Sources: GOC:ai Definition: Any process that decreases the concentration of calcium ions in mitochondria.